{
  "term_label": "cytoplasm",
  "gene_symbol": "RALGAPA2",
  "gene_name": "Ral GTPase-activating protein subunit alpha-2",
  "gene": "UniProtKB:Q2PPJ7",
  "term_id": "GO:0005737"
}